{
  "gene_symbol": "UBE3D",
  "term_label": "ubiquitin conjugating enzyme binding",
  "term_id": "GO:0031624",
  "gene": "UniProtKB:Q7Z6J8",
  "gene_name": "E3 ubiquitin-protein ligase E3D"
}